{
  "term_label": "Unknown biological process",
  "gene": "UniProtKB:Q8WYA6",
  "gene_name": "Beta-catenin-like protein 1",
  "term_id": "UNKNOWN:0002",
  "gene_symbol": "CTNNBL1"
}